{
  "gene_name": "Saccharopine dehydrogenase-like oxidoreductase",
  "term_id": "GO:0005811",
  "gene": "UniProtKB:Q8NBX0",
  "gene_symbol": "SCCPDH",
  "term_label": "lipid droplet"
}